presynaptic active zone membrane [GO:0048787] (cellular component) Definition: The membrane portion of the presynaptic active zone; it is the site where docking and fusion of synaptic vesicles occurs for the release of neurotransmitters. Also known as: active zone plasma membrane, active zone pre-synaptic plasma membrane, active zone presynaptic plasma membrane, pre-synaptic active zone membrane Relationships: is a type of GO:0097060; is part of presynaptic membrane [GO:0042734]; is part of presynaptic active zone [GO:0048786] References: PMID:12812759, PMID:12923177, PMID:3152289